{
  "gene_symbol": "FCN2",
  "gene_name": "Ficolin-2",
  "term_id": "GO:0031012",
  "gene": "UniProtKB:Q15485",
  "term_label": "extracellular matrix"
}